oocyte growth [GO:0001555] (biological process) Definition: The developmental growth process in which an oocyte irreversibly increases in size over time by accretion and biosynthetic production of matter similar to that already present. Sources: https://www.ncbi.nlm.nih.gov/books/NBK279054/ Subtypes: oocyte growth in germarium-derived egg chamber [GO:0030715] Relationships: is a type of developmental process involved in reproduction [GO:0003006]; is a type of developmental cell growth [GO:0048588]; BFO_0000050 oocyte development [GO:0048599]